{
  "gene_name": "Aurora kinase A and ninein-interacting protein",
  "gene": "UniProtKB:Q9H7T9",
  "term_label": "centrosome",
  "term_id": "GO:0005813",
  "gene_symbol": "AUNIP"
}